{
  "gene": "UniProtKB:Q86VW1",
  "term_label": "Unknown molecular function",
  "gene_name": "Solute carrier family 22 member 16",
  "term_id": "UNKNOWN:0001",
  "gene_symbol": "SLC22A16"
}